actomyosin contractile ring contraction [GO:0000916] (BP) Sources: GOC:clt, GOC:dph, GOC:mah, GOC:tb Also known as: cytokinesis, contractile ring contraction, actomyosin contractile ring constriction, contractile ring contraction involved in cell cycle cytokinesis, cytokinesis, actomyosin ring contraction Definition: The process of an actomyosin ring getting smaller in diameter, in the context of cytokinesis that takes place as part of a cell cycle. Subtypes: mitotic actomyosin contractile ring contraction [GO:1902404] Regulation: regulated by GO:0031991 Relationships: is a type of GO:0036213; is part of actomyosin contractile ring organization [GO:0044837]